{
  "gene_name": "Putative inactive beta-glucuronidase-like protein SMA3",
  "term_id": "UNKNOWN:0003",
  "gene_symbol": "GUSBP1",
  "term_label": "Unknown cellular component",
  "gene": "UniProtKB:Q15486"
}